nuclear proteasome regulatory particle, lid subcomplex [GO:0031613] (cellular component) Definition: The subunits that form the peripheral lid of the regulatory particle of a proteasome located in the nucleus of a cell. Sources: GOC:mah Relationships: is a type of GO:0008541; is a type of nuclear protein-containing complex [GO:0140513]; is part of nuclear proteasome regulatory particle [GO:0031598]